{
  "gene": "UniProtKB:Q6STE5",
  "gene_name": "SWI_SNF-related matrix-associated actin-dependent regulator of chromatin subfamily D member 3",
  "gene_symbol": "SMARCD3",
  "term_label": "regulation of transcription by RNA polymerase II",
  "term_id": "GO:0006357"
}